{
  "gene_symbol": "OR1L6",
  "term_label": "plasma membrane",
  "gene_name": "Olfactory receptor 1L6",
  "gene": "UniProtKB:Q8NGR2",
  "term_id": "GO:0005886"
}